{
  "gene_name": "Olfactory receptor 10G7",
  "term_label": "olfactory receptor activity",
  "gene": "UniProtKB:Q8NGN6",
  "gene_symbol": "OR10G7",
  "term_id": "GO:0004984"
}